{
  "gene": "UniProtKB:Q06136",
  "gene_name": "3-ketodihydrosphingosine reductase",
  "term_id": "GO:0047560",
  "term_label": "3-dehydrosphinganine reductase activity",
  "gene_symbol": "KDSR"
}